nutrient storage [GO:0170062] (biological process) Subtypes: lipid storage [GO:0019915], protein storage [GO:0140089] Sources: GOC:ew Definition: The accumulation and maintenance in cells or tissues of a nutrient, a substance that is used by an organism to survive, to grow, and to reproduce; such as proteins, vitamins, and minerals. Nutrient reserves can be accumulated for mobilization and utilization when needed. Relationships: is a type of cellular process [GO:0009987]